{
  "gene_name": "Integrin beta-2",
  "term_label": "integrin-mediated signaling pathway",
  "gene_symbol": "ITGB2",
  "gene": "UniProtKB:P05107",
  "term_id": "GO:0007229"
}